cytoplasmic side of nuclear pore [GO:1990876] (cellular component) References: PMID:8422679 Relationships: is a type of cellular anatomical structure [GO:0110165]; is part of nuclear pore [GO:0005643] Definition: The side of the nuclear pore complex (NPC) that faces the cytoplasm. Also known as: cytoplasmic side of NPC, cytoplasmic side of nuclear pore complex, cytoplasmic side of nucleopore